{
  "term_label": "cytoplasm",
  "gene": "UniProtKB:Q9NWW6",
  "gene_name": "Nicotinamide riboside kinase 1",
  "gene_symbol": "NMRK1",
  "term_id": "GO:0005737"
}